{
  "term_id": "GO:0030318",
  "term_label": "melanocyte differentiation",
  "gene": "UniProtKB:Q9H2I8",
  "gene_symbol": "LRMDA",
  "gene_name": "Leucine-rich melanocyte differentiation-associated protein"
}